{
  "term_label": "DNA-binding transcription factor activity, RNA polymerase II-specific",
  "term_id": "GO:0000981",
  "gene_symbol": "MYOD1",
  "gene_name": "Myoblast determination protein 1",
  "gene": "UniProtKB:P15172"
}